{
  "gene": "UniProtKB:P78324",
  "term_id": "GO:0005886",
  "gene_name": "Tyrosine-protein phosphatase non-receptor type substrate 1",
  "term_label": "plasma membrane",
  "gene_symbol": "SIRPA"
}